{
  "gene_symbol": "ZNF726P1",
  "gene_name": "Putative zinc finger protein 726P1",
  "gene": "UniProtKB:Q15940",
  "term_label": "RNA polymerase II cis-regulatory region sequence-specific DNA binding",
  "term_id": "GO:0000978"
}